{
  "term_id": "GO:0007018",
  "gene": "UniProtKB:Q9Y6G9",
  "gene_name": "Cytoplasmic dynein 1 light intermediate chain 1",
  "gene_symbol": "DYNC1LI1",
  "term_label": "microtubule-based movement"
}